{
  "gene_name": "Serpin B8",
  "gene_symbol": "SERPINB8",
  "term_label": "serine-type endopeptidase inhibitor activity",
  "gene": "UniProtKB:P50452",
  "term_id": "GO:0004867"
}